{
  "gene": "UniProtKB:Q8TDI7",
  "term_id": "GO:0005245",
  "gene_name": "Transmembrane channel-like protein 2",
  "term_label": "voltage-gated calcium channel activity",
  "gene_symbol": "TMC2"
}